{
  "gene": "UniProtKB:O95389",
  "term_label": "signal transduction",
  "gene_name": "Cellular communication network factor 6",
  "gene_symbol": "CCN6",
  "term_id": "GO:0007165"
}